{
  "gene_symbol": "XKRY",
  "gene_name": "Testis-specific XK-related protein, Y-linked",
  "gene": "UniProtKB:O14609",
  "term_id": "UNKNOWN:0003",
  "term_label": "Unknown cellular component"
}